{
  "term_label": "Unknown biological process",
  "gene": "UniProtKB:Q9BVW6",
  "gene_symbol": "SMIM2",
  "gene_name": "Small integral membrane protein 2",
  "term_id": "UNKNOWN:0002"
}